negative regulation of type 2 mitophagy [GO:1905090] (biological process) References: PMID:25009776, PMID:26942284 Sources: GOC:vw Definition: Any process that stops, prevents or reduces the frequency, rate or extent of type 2 mitophagy. Also known as: negative regulation of PRKN-mediated stimulation of mitophagy in response to mitochondrial depolarization, negative regulation of Park2-mediated stimulation of mitophagy in response to mitochondrial depolarization, negative regulation of parkin-mediated stimulation of mitophagy in response to mitochondrial depolarization Relationships: is a type of GO:1901525; is a type of regulation of type 2 mitophagy [GO:1905089]; negatively regulates type 2 mitophagy [GO:0061734]